{
  "term_label": "Unknown molecular function",
  "term_id": "UNKNOWN:0001",
  "gene_symbol": "DNAJC9-AS1",
  "gene": "UniProtKB:A6NH13",
  "gene_name": "Putative uncharacterized protein DNAJC9-AS1"
}